{
  "term_id": "GO:0007259",
  "term_label": "cell surface receptor signaling pathway via JAK-STAT",
  "gene": "UniProtKB:P42224",
  "gene_symbol": "STAT1",
  "gene_name": "Signal transducer and activator of transcription 1-alpha_beta"
}